{
  "term_id": "UNKNOWN:0001",
  "gene_symbol": "ATP6V1FNB",
  "gene_name": "Protein ATP6V1FNB",
  "term_label": "Unknown molecular function",
  "gene": "UniProtKB:A0A1B0GUX0"
}